regulation of growth hormone secretion [GO:0060123] (biological process) Definition: Any process that modulates the frequency, rate or extent of the regulated release of growth hormone from a cell. Sources: GOC:dph Relationships: is a type of regulation of peptide hormone secretion [GO:0090276]; regulates growth hormone secretion [GO:0030252] Subtypes: GO:0060124, GO:0060125